{
  "gene_symbol": "SYPL2",
  "term_id": "GO:0030672",
  "gene": "UniProtKB:Q5VXT5",
  "gene_name": "Synaptophysin-like protein 2",
  "term_label": "synaptic vesicle membrane"
}